positive regulation of skeletal muscle tissue regeneration [GO:0043415] (biological process) Definition: Any process that activates or increase the rate of skeletal muscle regeneration. Subtypes: GO:0014718 Also known as: up regulation of skeletal muscle regeneration, up-regulation of skeletal muscle regeneration, upregulation of skeletal muscle regeneration, activation of skeletal muscle regeneration, stimulation of skeletal muscle regeneration Sources: GOC:jl Relationships: is a type of GO:0043416; is a type of positive regulation of developmental growth [GO:0048639]; positively regulates skeletal muscle tissue regeneration [GO:0043403]